{
  "gene": "UniProtKB:Q9Y473",
  "term_label": "Unknown molecular function",
  "gene_name": "Zinc finger protein 175",
  "gene_symbol": "ZNF175",
  "term_id": "UNKNOWN:0001"
}